{
  "gene_name": "ATP-dependent translocase ABCB1",
  "term_label": "ATPase-coupled transmembrane transporter activity",
  "gene": "UniProtKB:P08183",
  "term_id": "GO:0042626",
  "gene_symbol": "ABCB1"
}